response to actinomycin D [GO:0072716] (biological process) Relationships: is a type of response to antibiotic [GO:0046677]; is a type of response to nitrogen compound [GO:1901698]; is a type of GO:1901700 Sources: GOC:mah Subtypes: cellular response to actinomycin D [GO:0072717] Definition: Any process that results in a change in state or activity of a cell or an organism (in terms of movement, secretion, enzyme production, gene expression, etc.) as a result of an actinomycin D stimulus.